{
  "gene_symbol": "CWH43",
  "term_label": "endoplasmic reticulum",
  "gene": "UniProtKB:Q9H720",
  "gene_name": "PGAP2-interacting protein",
  "term_id": "GO:0005783"
}